{
  "gene_symbol": "GSTM3",
  "gene": "UniProtKB:P21266",
  "gene_name": "Glutathione S-transferase Mu 3",
  "term_id": "GO:0004364",
  "term_label": "glutathione transferase activity"
}